{
  "gene_symbol": "MTRR",
  "gene": "UniProtKB:Q9UBK8",
  "gene_name": "Methionine synthase reductase",
  "term_label": "homocysteine metabolic process",
  "term_id": "GO:0050667"
}